{
  "gene": "UniProtKB:Q9NRU3",
  "term_id": "GO:0022857",
  "term_label": "transmembrane transporter activity",
  "gene_name": "Metal transporter CNNM1",
  "gene_symbol": "CNNM1"
}